{
  "gene_symbol": "ELAPOR1",
  "term_label": "plasma membrane",
  "term_id": "GO:0005886",
  "gene_name": "Endosome_lysosome-associated apoptosis and autophagy regulator 1",
  "gene": "UniProtKB:Q6UXG2"
}